{
  "gene_name": "GPN-loop GTPase 1",
  "term_id": "UNKNOWN:0002",
  "gene_symbol": "GPN1",
  "gene": "UniProtKB:Q9HCN4",
  "term_label": "Unknown biological process"
}